{
  "gene": "UniProtKB:Q9H013",
  "term_label": "metalloendopeptidase activity",
  "gene_symbol": "ADAM19",
  "gene_name": "Disintegrin and metalloproteinase domain-containing protein 19",
  "term_id": "GO:0004222"
}